{
  "term_label": "protein folding chaperone",
  "gene_name": "Heat shock 70 kDa protein 6",
  "gene": "UniProtKB:P17066",
  "term_id": "GO:0044183",
  "gene_symbol": "HSPA6"
}